{
  "gene": "UniProtKB:Q8N680",
  "term_id": "GO:0002682",
  "term_label": "regulation of immune system process",
  "gene_symbol": "ZBTB2",
  "gene_name": "Zinc finger and BTB domain-containing protein 2"
}